basic amino acid transmembrane export from vacuole [GO:0034488] (biological process) Relationships: is a type of amino acid transmembrane export from vacuole [GO:0032974]; is a type of vacuolar amino acid transmembrane transport [GO:0034487]; is a type of basic amino acid transmembrane transport [GO:1990822] Definition: The directed movement of basic amino acids out of the vacuole, across the vacuolar membrane. Sources: GOC:mah